cellular response to interleukin-7 [GO:0098761] (BP) Definition: Any process that results in a change in state or activity of a cell (in terms of movement, secretion, enzyme production, gene expression, etc.) as a result of an interleukin-7 stimulus. Relationships: is a type of GO:0071345; is_a response to interleukin-7 [GO:0098760] Also known as: cellular response to IL-7 Sources: GOC:BHF, GOC:mah